{
  "term_id": "UNKNOWN:0002",
  "gene_symbol": "CTDSP1",
  "term_label": "Unknown biological process",
  "gene": "UniProtKB:Q9GZU7",
  "gene_name": "Carboxy-terminal domain RNA polymerase II polypeptide A small phosphatase 1"
}